{
  "gene_symbol": "FGF8",
  "gene": "UniProtKB:P55075",
  "gene_name": "Fibroblast growth factor 8",
  "term_id": "GO:0009953",
  "term_label": "dorsal/ventral pattern formation"
}